{
  "term_id": "GO:0046471",
  "gene_symbol": "PLA2G2D",
  "term_label": "phosphatidylglycerol metabolic process",
  "gene": "UniProtKB:Q9UNK4",
  "gene_name": "Group IID secretory phospholipase A2"
}